{
  "term_label": "endomembrane system",
  "gene_name": "Membrane-associated progesterone receptor component 1",
  "gene": "UniProtKB:O00264",
  "term_id": "GO:0012505",
  "gene_symbol": "PGRMC1"
}